{
  "gene_name": "HLA class I histocompatibility antigen, C alpha chain",
  "term_id": "GO:0005615",
  "gene": "UniProtKB:P10321",
  "gene_symbol": "HLA-C",
  "term_label": "extracellular space"
}